very long-chain fatty acyl-CoA hydrolase activity [GO:0052817] (molecular function) Definition: Catalysis of the reaction: a very long-chain fatty acyl-CoA + H2O = a very long-chain fatty acid + CoA + H+. A very long-chain fatty acid has an aliphatic tail containing more than 22 carbons. Relationships: is a type of GO:0047617 Sources: RHEA:67072 Note: While there is not universal consensus on the lengths of short-, medium-, long- and very-long-chain fatty acids, the GO uses the definitions in ChEBI (see CHEBI:26666, CHEBI:59554, CHEBI:15904 and CHEBI:27283). Also known as: very long-chain acyl coenzyme A hydrolase activity, very long-chain acyl-thioester hydrolase activity, very long-chain hydrolase activity, very long-chain-acyl-CoA hydrolase activity